trigeminal nerve formation [GO:0021638] (biological process) Definition: The process that gives rise to the trigeminal nerve. This process pertains to the initial formation of a structure from unspecified parts. The trigeminal nerve is composed of three large branches. They are the ophthalmic (V1, sensory), maxillary (V2, sensory) and mandibular (V3, motor and sensory) branches. The sensory ophthalmic branch travels through the superior orbital fissure and passes through the orbit to reach the skin of the forehead and top of the head. The maxillary nerve contains sensory branches that reach the pterygopalatine fossa via the inferior orbital fissure (face, cheek and upper teeth) and pterygopalatine canal (soft and hard palate, nasal cavity and pharynx). The motor part of the mandibular branch is distributed to the muscles of mastication, the mylohyoid muscle and the anterior belly of the digastric. The mandibular nerve also innervates the tensor veli palatini and tensor tympani muscles. The sensory part of the mandibular nerve is composed of branches that carry general sensory information from the mucous membranes of the mouth and cheek, anterior two-thirds of the tongue, lower teeth, skin of the lower jaw, side of the head and scalp and meninges of the anterior and middle cranial fossae. Sources: GOC:cls, GOC:dgh, GOC:dph, GOC:jid, GO_REF:0000021 Also known as: CN V biosynthesis, CN V formation Relationships: is a type of cranial nerve formation [GO:0021603]; is part of GO:0021636